{
  "term_label": "Unknown biological process",
  "term_id": "UNKNOWN:0002",
  "gene_symbol": "PPP1R14D",
  "gene": "UniProtKB:Q9NXH3",
  "gene_name": "Protein phosphatase 1 regulatory subunit 14D"
}